negative regulation of erythrocyte aggregation [GO:0034119] (biological process) Definition: Any process that stops, prevents, or reduces the frequency, rate, or extent of erythrocyte aggregation. Also known as: negative regulation of RBC aggregation, negative regulation of red blood cell aggregation Sources: GOC:add Relationships: is a type of negative regulation of homotypic cell-cell adhesion [GO:0034111]; is a type of GO:0034118; negatively regulates GO:0034117